{
  "gene": "UniProtKB:Q8WTV0",
  "gene_symbol": "SCARB1",
  "term_id": "GO:0043654",
  "term_label": "recognition of apoptotic cell",
  "gene_name": "Scavenger receptor class B member 1"
}